{
  "gene": "UniProtKB:Q75N03",
  "term_id": "GO:0016567",
  "gene_symbol": "CBLL1",
  "gene_name": "E3 ubiquitin-protein ligase Hakai",
  "term_label": "protein ubiquitination"
}